MKS complex [GO:0036038] (cellular component) Definition: A protein complex that is located at the ciliary transition zone and consists of several proteins some of which are membrane bound. Acts as an organiser of transition zone inner structure, specifically the Y-shaped links, in conjunction with the NPHP complex. The MKS complex also acts as part of the selective barrier that prevents diffusion of proteins between the ciliary cytoplasm and cellular cytoplasm as well as between the ciliary membrane and plasma membrane. References: PMID:21422230, PMID:21565611, PMID:21725307, PMID:22179047, PMID:25869670, PMID:26595381, PMID:26982032 Sources: GOC:cilia, GOC:sp Note: Although there is some evidence, it is still unclear if the MKS and NPHP complexes are constituents parts of the Y-shaped links or are simply responsible for aligning and attaching the Y-shaped links to the membrane and axoneme. Relationships: is a type of GO:0032991; BFO_0000050 GO:0035869 Also known as: TCTN-B9D complex, MKS module, B9 complex, tectonic complex, tectonic-like complex